{
  "gene_name": "Pancreas transcription factor 1 subunit alpha",
  "term_label": "DNA-binding transcription factor activity, RNA polymerase II-specific",
  "term_id": "GO:0000981",
  "gene": "UniProtKB:Q7RTS3",
  "gene_symbol": "PTF1A"
}